{
  "gene": "UniProtKB:Q9ULW3",
  "gene_symbol": "ABT1",
  "term_id": "GO:0005730",
  "term_label": "nucleolus",
  "gene_name": "Activator of basal transcription 1"
}